regulation of tolerance induction to tumor cell [GO:0002843] (biological process) Definition: Any process that modulates the frequency, rate, or extent of tolerance induction to tumor cell. Sources: GOC:add Also known as: regulation of tolerance induction to tumour cell Relationships: is a type of regulation of peripheral tolerance induction [GO:0002658]; is a type of regulation of immune response to tumor cell [GO:0002837]; regulates tolerance induction to tumor cell [GO:0002413] Subtypes: negative regulation of tolerance induction to tumor cell [GO:0002844], positive regulation of tolerance induction to tumor cell [GO:0002845], regulation of T cell tolerance induction to tumor cell [GO:0002846]